cerebellar neuron development [GO:0098749] (biological process) Regulation: regulated by regulation of cerebellar neuron development [GO:1905079]; negatively regulated by negative regulation of cerebellar neuron development [GO:1905080]; positively regulated by positive regulation of cerebellar neuron development [GO:1905081] Sources: GOC:dos Relationships: is a type of central nervous system neuron development [GO:0021954]; is part of GO:0021549 Definition: The process whose specific outcome is the progression of a cerebellar neuron over time, from initial commitment of the cell to a specific fate, to the fully functional differentiated cell.